cucurbitadienol synthase activity [GO:0034076] (molecular function) Relationships: is a type of oxidosqualene cyclase activity [GO:0031559] Definition: Catalysis of the reaction: oxidosqualene = cucurbitadienol. References: PMID:18033581 Sources: GOC:cb